{
  "term_label": "DNA-directed DNA polymerase activity",
  "term_id": "GO:0003887",
  "gene": "UniProtKB:Q9Y253",
  "gene_name": "DNA polymerase eta",
  "gene_symbol": "POLH"
}